positive regulation of brassinosteroid mediated signaling pathway [GO:1900459] (biological process) References: PMID:21855796 Sources: GOC:TermGenie Relationships: is a type of positive regulation of signal transduction [GO:0009967]; is a type of regulation of brassinosteroid mediated signaling pathway [GO:1900457]; positively regulates brassinosteroid mediated signaling pathway [GO:0009742] Definition: Any process that activates or increases the frequency, rate or extent of brassinosteroid mediated signaling pathway. Also known as: activation of brassinosteroid mediated signalling, positive regulation of brassinosteroid mediated signalling, up regulation of brassinosteroid mediated signaling pathway, up regulation of brassinosteroid mediated signalling, up-regulation of brassinosteroid mediated signaling pathway, up-regulation of brassinosteroid mediated signalling, upregulation of brassinosteroid mediated signaling pathway, upregulation of brassinosteroid mediated signalling, activation of brassinosteroid mediated signaling pathway